{
  "gene_symbol": "EFCAB13",
  "term_id": "UNKNOWN:0001",
  "term_label": "Unknown molecular function",
  "gene": "UniProtKB:Q8IY85",
  "gene_name": "EF-hand calcium-binding domain-containing protein 13"
}